plasma membrane raft assembly [GO:0044854] (biological process) Subtypes: GO:0070836 Definition: The aggregation, arrangement and bonding together of a set of components to form a plasma membrane raft. Sources: GOC:jl Relationships: is a type of membrane raft assembly [GO:0001765]; is a type of GO:0044857